{
  "term_id": "GO:0005615",
  "gene_name": "Intelectin-1",
  "term_label": "extracellular space",
  "gene_symbol": "ITLN1",
  "gene": "UniProtKB:Q8WWA0"
}